{
  "term_id": "GO:0006893",
  "term_label": "Golgi to plasma membrane transport",
  "gene_name": "Exocyst complex component 6B",
  "gene_symbol": "EXOC6B",
  "gene": "UniProtKB:Q9Y2D4"
}